{
  "gene": "UniProtKB:Q99547",
  "term_id": "GO:0000460",
  "term_label": "maturation of 5.8S rRNA",
  "gene_symbol": "MPHOSPH6",
  "gene_name": "M-phase phosphoprotein 6"
}